{
  "gene_symbol": "KISS1R",
  "term_id": "GO:0046887",
  "term_label": "positive regulation of hormone secretion",
  "gene": "UniProtKB:Q969F8",
  "gene_name": "KiSS-1 receptor"
}